dopamine uptake involved in synaptic transmission [GO:0051583] (BP) Definition: The directed movement of dopamine into a presynaptic neuron or glial cell. In this context, dopamine is a catecholamine neurotransmitter and a metabolic precursor of noradrenaline and adrenaline. Regulation: regulated by GO:0051584; negatively regulated by negative regulation of dopamine uptake involved in synaptic transmission [GO:0051585]; positively regulated by GO:0051586 Also known as: dopamine import involved in synaptic transmission, dopamine reuptake involved in synaptic transmission Sources: GOC:ai Relationships: is a type of catecholamine uptake involved in synaptic transmission [GO:0051934]; is a type of dopamine uptake [GO:0090494]; is part of synaptic transmission, dopaminergic [GO:0001963]